regulation of Schwann cell proliferation [GO:0010624] (biological process) Subtypes: positive regulation of Schwann cell proliferation [GO:0010625], GO:0010626, GO:1905044 Sources: GOC:dph, GOC:sl, GOC:tb Definition: Any process that modulates the frequency or rate of multiplication or reproduction of Schwann cells, resulting in the expansion of their population. Schwann cells are a type of glial cell in the peripheral nervous system. Relationships: is a type of regulation of glial cell proliferation [GO:0060251]; regulates GO:0014010